{
  "gene": "UniProtKB:Q9H0I2",
  "gene_symbol": "ENKD1",
  "term_label": "Unknown molecular function",
  "term_id": "UNKNOWN:0001",
  "gene_name": "Enkurin domain-containing protein 1"
}